endospore-forming forespore [GO:0042601] (cellular component) Definition: Portion of the cell formed during the process of bacterial sporulation that will ultimately become the core of the endospore. An endospore is a type of dormant cell that is resistant to adverse conditions. Sources: GOC:jl, GOC:mtg_sensu, ISBN:0697286029 Relationships: is a type of intracellular immature spore [GO:0042763]